mitochondrial S-adenosyl-L-methionine transmembrane transport [GO:1990543] (biological process) Definition: The process in which S-adenosyl-L-methionine is transported across a mitochondrial membrane, into or out of the mitochondrion. References: PMID:14609944 Relationships: is_a GO:1901962